sperm mitochondrion organization [GO:0030382] (biological process) References: PMID:8833144 Sources: GOC:dph, GOC:jl, GOC:mah Definition: A process that is carried out at the cellular level which results in the assembly, arrangement of constituent parts, or disassembly of sperm mitochondria; the process in which they take on their characteristic morphology; they are flattened, elongated, and arranged circumferentially into a tight helical coil around the tail-dense fibers of the mature sperm. Relationships: is a type of mitochondrion organization [GO:0007005] Also known as: sperm mitochondria organisation, sperm mitochondria organization and biogenesis, sperm mitochondrion organization and biogenesis